{
  "gene": "UniProtKB:Q96GA3",
  "gene_symbol": "LTV1",
  "gene_name": "Protein LTV1 homolog",
  "term_id": "GO:0005634",
  "term_label": "nucleus"
}